{
  "gene_symbol": "CTDSPL2",
  "term_label": "phosphoprotein phosphatase activity",
  "gene_name": "CTD small phosphatase-like protein 2",
  "term_id": "GO:0004721",
  "gene": "UniProtKB:Q05D32"
}